formate dehydrogenase complex [GO:0009326] (cellular component) Definition: An enzyme complex that catalyzes the dehydrogenation of formate to produce carbon dioxide (CO2). References: PMID:1504073, PMID:8566699 Relationships: is_a oxidoreductase complex [GO:1990204]